{
  "gene_name": "E3 ubiquitin-protein ligase TRAF7",
  "gene_symbol": "TRAF7",
  "gene": "UniProtKB:Q6Q0C0",
  "term_label": "Unknown molecular function",
  "term_id": "UNKNOWN:0001"
}